general transcription initiation factor activity [GO:0140223] (molecular function) Note: Usage guidance: The distinction between general transcription factors and DNA-binding transcription factors is that the latter modulate the selection of which genes are expressed under specific conditions, while general transcription factors are the constitutive machinery required for transcription initiation. Relationships: is a type of molecular_function [GO:0003674]; is part of DNA-templated transcription [GO:0006351] Subtypes: RNA polymerase III general transcription initiation factor activity [GO:0000995], RNA polymerase I general transcription initiation factor activity [GO:0001181], RNA polymerase II general transcription initiation factor activity [GO:0016251], mitochondrial RNA polymerase general transcription initiation factor activity [GO:0180066] Sources: GOC:txnOH-2018 Also known as: GTF activity, basal transcription factor activity, general transcription factor activity Definition: A molecular function required for core promoter activity that mediates the assembly of the RNA polymerase holoenzyme at promoter DNA to form the pre-initiation complex (PIC). General transcription factors (GTFs) bind to and open promoter DNA, initiate RNA synthesis and stimulate the escape of the polymerase from the promoter. Not all subunits of the general transcription factor are necessarily present at all promoters to initiate transcription. GTFs act at each promoter, although the exact subunit composition at individual promoters may vary.